{
  "term_id": "GO:0004807",
  "gene_name": "Triosephosphate isomerase",
  "gene": "UniProtKB:P60174",
  "gene_symbol": "TPI1",
  "term_label": "triose-phosphate isomerase activity"
}